{
  "gene_name": "Inter-alpha-trypsin inhibitor heavy chain H6",
  "term_id": "UNKNOWN:0003",
  "term_label": "Unknown cellular component",
  "gene_symbol": "ITIH6",
  "gene": "UniProtKB:Q6UXX5"
}